{
  "gene_symbol": "FOXJ2",
  "term_id": "GO:0000978",
  "term_label": "RNA polymerase II cis-regulatory region sequence-specific DNA binding",
  "gene": "UniProtKB:Q9P0K8",
  "gene_name": "Forkhead box protein J2"
}